{
  "gene_name": "Phosphatidylcholine:ceramide cholinephosphotransferase 2",
  "gene": "UniProtKB:Q8NHU3",
  "term_label": "sphingomyelin biosynthetic process",
  "term_id": "GO:0006686",
  "gene_symbol": "SGMS2"
}